positive regulation of peptide hormone processing [GO:0060569] (biological process) Definition: Any process that increases the rate, frequency or extent of peptide hormone processing. Peptide hormone processing is the generation of a mature peptide hormone by posttranslational processing of a prohormone. Relationships: is a type of positive regulation of protein processing [GO:0010954]; is a type of GO:0032352; is a type of GO:0034250; is a type of GO:0060568; RO_0002213 peptide hormone processing [GO:0016486] Sources: GOC:dph, GOC:tb